protein-N(PI)-phosphohistidine-lactose phosphotransferase system transporter activity [GO:0022869] (molecular function) Relationships: is a type of protein-N(PI)-phosphohistidine-sugar phosphotransferase activity [GO:0008982]; is a type of lactose transmembrane transporter activity [GO:0015155] Sources: GOC:mtg_transport, ISBN:0815340729 Definition: Catalysis of the PEP-dependent, phosphoryl transfer-driven transport of substances across a membrane. The transport happens by catalysis of the reaction: protein N-phosphohistidine + lactose(out) = protein histidine + lactose phosphate(in). This differs from primary and secondary active transport in that the solute is modified during transport. Also known as: lactose PTS transporter activity